regulation of dense core granule exocytosis [GO:1905413] (biological process) Definition: Any process that modulates the frequency, rate or extent of dense core granule exocytosis. Subtypes: regulation of presynaptic dense core granule exocytosis [GO:0099161], regulation of postsynaptic dense core vesicle exocytosis [GO:0150044], negative regulation of dense core granule exocytosis [GO:1905414], GO:1905415 Also known as: regulation of dense core vesicle exocytosis Relationships: is a type of GO:0017158; occurs in presynapse [GO:0098793]; regulates dense core granule exocytosis [GO:1990504] References: PMID:18468511 Sources: GOC:PARL, GOC:TermGenie, GOC:bf, GO_REF:0000058